{
  "gene_symbol": "RUVBL1",
  "gene_name": "RuvB-like 1",
  "gene": "UniProtKB:Q9Y265",
  "term_label": "Ino80 complex",
  "term_id": "GO:0031011"
}